{
  "term_id": "GO:0045944",
  "gene_name": "Nuclear receptor subfamily 1 group I member 2",
  "gene": "UniProtKB:O75469",
  "gene_symbol": "NR1I2",
  "term_label": "positive regulation of transcription by RNA polymerase II"
}